p-xylene catabolic process [GO:0042187] (biological process) Also known as: p-xylene breakdown, p-xylene catabolism, p-xylene degradation, para-xylene catabolic process, para-xylene catabolism Sources: GOC:jl Definition: The chemical reactions and pathways resulting in the breakdown of p-xylene (1,4-dimethylbenzene), a colorless, liquid aromatic hydrocarbon. Relationships: is_a xylene catabolic process [GO:0042184]